negative regulation of sensory neuron axon guidance [GO:1905490] (biological process) Also known as: down regulation of sensory neuron axon guidance, down-regulation of sensory neuron axon guidance, downregulation of sensory neuron axon guidance, inhibition of sensory neuron axon guidance Relationships: is a type of negative regulation of axon guidance [GO:1902668]; is a type of regulation of sensory neuron axon guidance [GO:1905489]; negatively regulates sensory neuron axon guidance [GO:0097374] References: PMID:16516839 Sources: GOC:TermGenie, GO_REF:0000058 Definition: Any process that stops, prevents or reduces the frequency, rate or extent of sensory neuron axon guidance.